negative regulation of intracellular transport [GO:0032387] (BP) Relationships: is a type of regulation of intracellular transport [GO:0032386]; is a type of negative regulation of cellular process [GO:0048523]; is a type of GO:0051051; negatively regulates intracellular transport [GO:0046907] Sources: GOC:mah Definition: Any process that stops, prevents, or reduces the frequency, rate or extent of the directed movement of substances within cells. Also known as: down regulation of intracellular transport, down-regulation of intracellular transport, downregulation of intracellular transport, inhibition of intracellular transport Subtypes: GO:0032378, negative regulation of nucleocytoplasmic transport [GO:0046823], negative regulation of anterograde axonal transport of mitochondrion [GO:0061882], negative regulation of intracellular protein transport [GO:0090317], negative regulation of cargo loading into COPII-coated vesicle [GO:1901303], negative regulation of vesicle transport along microtubule [GO:1901609], negative regulation of calcium ion import into sarcoplasmic reticulum [GO:1902081], GO:1902839, GO:1903336, GO:1904810, negative regulation of retrograde transport, endosome to Golgi [GO:1905280], negative regulation of intraciliary anterograde transport [GO:1905797], negative regulation of intraciliary retrograde transport [GO:1905800], negative regulation of early endosome to late endosome transport [GO:2000642], GO:2001018, negative regulation of endocytic recycling [GO:2001136]